zinc ion import into organelle [GO:0062111] (biological process) Relationships: is a type of GO:0071577 Definition: The directed import of zinc(2+) from the cytosol, across an organelle membrane, into the organelle. Subtypes: zinc ion import into synaptic vesicle [GO:0099180], zinc ion import into endoplasmic reticulum [GO:0140209], zinc ion import into secretory vesicle [GO:0140914], zinc ion import into lysosome [GO:0140916], zinc ion import into mitochondrion [GO:0140917], zinc ion import into Golgi lumen [GO:1904257] References: PMID:29529046